{
  "gene_name": "Deoxyguanosine kinase, mitochondrial",
  "term_id": "GO:0005737",
  "gene": "UniProtKB:Q16854",
  "term_label": "cytoplasm",
  "gene_symbol": "DGUOK"
}